{
  "gene_symbol": "NCKAP1L",
  "term_label": "Unknown molecular function",
  "gene": "UniProtKB:P55160",
  "term_id": "UNKNOWN:0001",
  "gene_name": "Nck-associated protein 1-like"
}